{
  "term_id": "GO:0006508",
  "gene_symbol": "PRSS56",
  "term_label": "proteolysis",
  "gene": "UniProtKB:P0CW18",
  "gene_name": "Serine protease 56"
}